plasmodesma [GO:0009506] (cellular component) Also known as: plasmodesmata Subtypes: primary plasmodesma [GO:0009550], GO:0009551 References: PMID:29880547 Definition: A fine cytoplasmic channel, found in all higher plants, that connects the cytoplasm of one cell to that of an adjacent cell. Relationships: is a type of cell-cell junction [GO:0005911]; BFO_0000050 GO:0055044